{
  "term_label": "proteasome-mediated ubiquitin-dependent protein catabolic process",
  "gene_name": "Kelch-like protein 36",
  "term_id": "GO:0043161",
  "gene_symbol": "KLHL36",
  "gene": "UniProtKB:Q8N4N3"
}